{
  "term_label": "Unknown biological process",
  "term_id": "UNKNOWN:0002",
  "gene_name": "G patch domain-containing protein 2-like",
  "gene": "UniProtKB:Q9NWQ4",
  "gene_symbol": "GPATCH2L"
}